{
  "gene_name": "Olfactory receptor 8S1",
  "term_id": "GO:0007165",
  "term_label": "signal transduction",
  "gene": "UniProtKB:Q8NH09",
  "gene_symbol": "OR8S1"
}